{
  "gene_name": "Proteasome subunit beta type-5",
  "term_label": "proteasome-mediated ubiquitin-dependent protein catabolic process",
  "gene_symbol": "PSMB5",
  "term_id": "GO:0043161",
  "gene": "UniProtKB:P28074"
}